{
  "gene_name": "Inactive rhomboid protein 1",
  "gene_symbol": "RHBDF1",
  "term_label": "endoplasmic reticulum membrane",
  "gene": "UniProtKB:Q96CC6",
  "term_id": "GO:0005789"
}